{
  "term_label": "plasma membrane",
  "gene": "UniProtKB:O14817",
  "gene_name": "Tetraspanin-4",
  "gene_symbol": "TSPAN4",
  "term_id": "GO:0005886"
}